{
  "term_id": "GO:0048704",
  "gene_symbol": "HOXA4",
  "gene_name": "Homeobox protein Hox-A4",
  "gene": "UniProtKB:Q00056",
  "term_label": "embryonic skeletal system morphogenesis"
}